{
  "gene_name": "F-box_LRR-repeat protein 14",
  "term_label": "Unknown molecular function",
  "gene": "UniProtKB:Q8N1E6",
  "term_id": "UNKNOWN:0001",
  "gene_symbol": "FBXL14"
}